{
  "term_id": "UNKNOWN:0001",
  "gene_name": "LBH domain-containing protein 2",
  "gene": "UniProtKB:A0A0U1RRK4",
  "gene_symbol": "LBHD2",
  "term_label": "Unknown molecular function"
}